superoxide reductase activity [GO:0050605] (molecular function) Definition: Catalysis of the reaction: superoxide + reduced rubredoxin + 2 H+ = H2O2 + rubredoxin. Sources: EC:1.15.1.2, MetaCyc:1.15.1.2-RXN Also known as: desulfoferrodoxin activity, neelaredoxin activity, rubredoxin:superoxide oxidoreductase activity Relationships: is a type of antioxidant activity [GO:0016209]; is a type of oxidoreductase activity, acting on superoxide radicals as acceptor [GO:0016721]